{
  "gene_symbol": "MTUS2",
  "term_id": "GO:0005634",
  "gene_name": "Microtubule-associated tumor suppressor candidate 2",
  "term_label": "nucleus",
  "gene": "UniProtKB:Q5JR59"
}